{
  "gene_symbol": "VPS18",
  "gene_name": "Vacuolar protein sorting-associated protein 18 homolog",
  "term_label": "endosome",
  "gene": "UniProtKB:Q9P253",
  "term_id": "GO:0005768"
}